{
  "gene_symbol": "DEFB116",
  "gene": "UniProtKB:Q30KQ4",
  "gene_name": "Beta-defensin 116",
  "term_label": "Unknown biological process",
  "term_id": "UNKNOWN:0002"
}